behavioral response to water deprivation [GO:0042630] (biological process) Relationships: is a type of behavior [GO:0007610]; is part of response to water deprivation [GO:0009414] Definition: Any process that results in a change in the behavior of an organism as a result of deprivation of water. Sources: GOC:jl Also known as: behavioral response to drought, behavioral response to thirst, behavioural response to water deprivation